{
  "gene_symbol": "IL13",
  "gene": "UniProtKB:P35225",
  "gene_name": "Interleukin-13",
  "term_label": "inflammatory response",
  "term_id": "GO:0006954"
}